demethoxycurcumin synthase activity [GO:0102103] (molecular function) Definition: Catalysis of the reaction: (4-coumaroyl)acetyl-CoA + 4-coumaryl-CoA + H2O = bisdemethoxycurcumin + 2 coenzyme A + carbon dioxide. Sources: EC:2.3.1.219 Relationships: is a type of acyltransferase activity, transferring groups other than amino-acyl groups [GO:0016747]